positive regulation of vascular endothelial cell proliferation [GO:1905564] (biological process) References: PMID:23201774 Sources: GOC:BHF, GOC:BHF_telomere, GOC:TermGenie, GOC:nc, GO_REF:0000058 Relationships: is a type of positive regulation of endothelial cell proliferation [GO:0001938]; is a type of regulation of vascular endothelial cell proliferation [GO:1905562]; positively regulates vascular endothelial cell proliferation [GO:0101023] Also known as: up regulation of vascular endothelial cell proliferation, up-regulation of vascular endothelial cell proliferation, upregulation of vascular endothelial cell proliferation, activation of vascular endothelial cell proliferation Definition: Any process that activates or increases the frequency, rate or extent of vascular endothelial cell proliferation.